pyrimidine nucleobase salvage [GO:0043100] (biological process) Also known as: pyrimidine base salvage Relationships: is a type of pyrimidine-containing compound salvage [GO:0008655]; is a type of GO:0019856 Sources: GOC:jl Definition: Any process that generates pyrimidine nucleobases, 1,3-diazine organic nitrogenous bases, from derivatives of them without de novo synthesis. Subtypes: GO:0006223